{
  "gene_symbol": "FAM151A",
  "term_label": "extracellular space",
  "gene_name": "Protein FAM151A",
  "gene": "UniProtKB:Q8WW52",
  "term_id": "GO:0005615"
}